H4/H2A histone acetyltransferase complex [GO:0043189] (cellular component) Also known as: H4/H2A HAT complex Sources: GOC:mah, GOC:rb Relationships: is a type of H4 histone acetyltransferase complex [GO:1902562] Subtypes: GO:0035267 Definition: A multisubunit complex that catalyzes the acetylation of histones H4 and H2A.